{
  "gene": "UniProtKB:P29474",
  "term_label": "response to hormone",
  "term_id": "GO:0009725",
  "gene_name": "Nitric oxide synthase 3",
  "gene_symbol": "NOS3"
}